{
  "term_id": "UNKNOWN:0001",
  "gene_symbol": "CHCHD3",
  "term_label": "Unknown molecular function",
  "gene_name": "MICOS complex subunit MIC19",
  "gene": "UniProtKB:Q9NX63"
}